{
  "term_id": "GO:0003682",
  "gene_symbol": "HMGN1",
  "gene": "UniProtKB:P05114",
  "term_label": "chromatin binding",
  "gene_name": "Non-histone chromosomal protein HMG-14"
}